{
  "gene_name": "EEIG family member 2",
  "gene_symbol": "EEIG2",
  "gene": "UniProtKB:Q5T8I3",
  "term_label": "Unknown cellular component",
  "term_id": "UNKNOWN:0003"
}